{
  "term_id": "GO:0005694",
  "gene_symbol": "SETD7",
  "gene_name": "Histone-lysine N-methyltransferase SETD7",
  "term_label": "chromosome",
  "gene": "UniProtKB:Q8WTS6"
}